{
  "gene_name": "Kinesin-like protein KIF1C",
  "term_id": "GO:0008017",
  "gene_symbol": "KIF1C",
  "term_label": "microtubule binding",
  "gene": "UniProtKB:O43896"
}